{
  "term_label": "semaphorin receptor activity",
  "gene_name": "Plexin-C1",
  "gene_symbol": "PLXNC1",
  "gene": "UniProtKB:O60486",
  "term_id": "GO:0017154"
}